tissue migration [GO:0090130] (biological process) Subtypes: mesoderm migration involved in gastrulation [GO:0007509], GO:0090131, epithelium migration [GO:0090132] Definition: The process in which the population of cells that make up a tissue undergo directed movement. Relationships: is a type of multicellular organismal process [GO:0032501] Sources: GOC:ascb_2009, GOC:dph, GOC:tb